{
  "term_id": "UNKNOWN:0001",
  "gene_symbol": "VXN",
  "gene": "UniProtKB:Q8TAG6",
  "gene_name": "Vexin",
  "term_label": "Unknown molecular function"
}